negative regulation of ecdysteroid secretion [GO:0045999] (BP) Sources: GOC:go_curators Definition: Any process that stops, prevents, or reduces the frequency, rate or extent of the regulated release of ecdysteroid. Also known as: down regulation of ecdysteroid secretion, down-regulation of ecdysteroid secretion, downregulation of ecdysteroid secretion, inhibition of ecdysteroid secretion Relationships: is a type of regulation of ecdysteroid secretion [GO:0007555]; is a type of negative regulation of steroid hormone secretion [GO:2000832]; negatively regulates ecdysteroid secretion [GO:0045457]